2-chloroacrylate reductase activity [GO:0102523] (MF) Sources: EC:1.3.1.103, GOC:pz Definition: Catalysis of the reaction: (S)-2-chloropropanoate + NADP = 2-chloroacrylate + NADPH + H+. Relationships: is a type of oxidoreductase activity, acting on the CH-CH group of donors, NAD or NADP as acceptor [GO:0016628]